L-phosphoserine phosphatase activity [GO:0036424] (molecular function) Also known as: O-phosphoserine phosphohydrolase activity, phosphoserine phosphatase activity References: PMID:25037224, PMID:9188776 Sources: RHEA:21208 Definition: Catalysis of the reaction: O-phospho-L-serine + H2O = L-serine + phosphate, on a free amino acid. Note: Do not confuse with protein phosphatases. For protein phosphatases, consider GO:0004722 ; protein serine/threonine phosphatase activity or GO:0008138 ; protein tyrosine/serine/threonine phosphatase activity. Relationships: is a type of phosphatase activity [GO:0016791]